{
  "term_label": "transmembrane signaling receptor activity",
  "term_id": "GO:0004888",
  "gene_symbol": "KIR2DL5B",
  "gene": "UniProtKB:Q8NHK3",
  "gene_name": "Killer cell immunoglobulin-like receptor 2DL5B"
}